de novo centriole assembly via blepharoplast [GO:0097743] (biological process) References: PMID:25047614 Sources: GOC:cilia Also known as: multiciliation, multiciliogenesis Relationships: is a type of GO:0097742 Definition: A de novo centriole assembly process observed in multi-ciliated sperm cells of some primitive land plants, and where centrioles are formed from a blepharoplast, ultimately giving rise to multiple cilia on the sperm surface.